protein K33-linked deubiquitination [GO:1990168] (biological process) Definition: A protein deubiquitination process in which a K33-linked ubiquitin chain, i.e. a polymer of ubiquitin formed by linkages between lysine residues at position 33 of the ubiquitin monomers, is removed from a protein. Relationships: is a type of protein deubiquitination [GO:0016579] References: PMID:23827681